regulation of activated CD4-positive, alpha-beta T cell apoptotic process [GO:1905399] (biological process) Subtypes: negative regulation of activated CD4-positive, alpha-beta T cell apoptotic process [GO:1905400], GO:1905401 References: PMID:24187568 Sources: GOC:TermGenie, GO_REF:0000058 Also known as: regulation of activated CD4-positive, alpha-beta T lymphocyte apoptotic process, regulation of activated CD4-positive, alpha-beta T-cell apoptotic process, regulation of activated CD4-positive, alpha-beta T-lymphocyte apoptotic process, regulation of activated CD4-positive, alpha-beta T cell apoptosis, regulation of activated CD4-positive, alpha-beta T lymphocyte apoptosis, regulation of activated CD4-positive, alpha-beta T-cell apoptosis, regulation of activated CD4-positive, alpha-beta T-lymphocyte apoptosis Relationships: is a type of GO:0070232; regulates GO:1905398 Definition: Any process that modulates the frequency, rate or extent of activated CD4-positive, alpha-beta T cell apoptotic process.